{
  "gene": "UniProtKB:Q6XYB7",
  "term_id": "GO:0000981",
  "term_label": "DNA-binding transcription factor activity, RNA polymerase II-specific",
  "gene_name": "Transcription factor LBX2",
  "gene_symbol": "LBX2"
}